{
  "gene": "UniProtKB:P13385",
  "term_label": "determination of left/right symmetry",
  "gene_name": "Teratocarcinoma-derived growth factor 1",
  "gene_symbol": "TDGF1",
  "term_id": "GO:0007368"
}